{
  "term_id": "GO:0003677",
  "gene_name": "ATPase family AAA domain-containing protein 5",
  "gene_symbol": "ATAD5",
  "term_label": "DNA binding",
  "gene": "UniProtKB:Q96QE3"
}